{
  "term_id": "UNKNOWN:0002",
  "term_label": "Unknown biological process",
  "gene_symbol": "LOC105372440",
  "gene_name": "Uncharacterized protein",
  "gene": "UniProtKB:A0A1B0GTG8"
}